{
  "gene_symbol": "GPX2",
  "gene": "UniProtKB:P18283",
  "term_label": "glutathione peroxidase activity",
  "term_id": "GO:0004602",
  "gene_name": "Glutathione peroxidase 2"
}